{
  "gene_symbol": "TRAV41",
  "term_label": "Unknown molecular function",
  "term_id": "UNKNOWN:0001",
  "gene": "UniProtKB:A0A0B4J266",
  "gene_name": "T cell receptor alpha variable 41"
}